SKA complex [GO:0170027] (cellular component) Definition: An outer kinetochore complex involved in the attachment of microtubule ends to the chromosomes during mitosis. In humans, it contains the subunits SKA1, SKA2 and SKA3. Also known as: SKA1 complex References: PMID:19289083, PMID:22483620 Relationships: is a type of protein-containing complex [GO:0032991]; is part of GO:0000940